{
  "gene": "UniProtKB:H7BZ55",
  "gene_name": "Ciliary rootlet coiled-coil protein 2",
  "gene_symbol": "CROCC2",
  "term_label": "centriole",
  "term_id": "GO:0005814"
}